response to methylamine [GO:0036255] (biological process) Relationships: is a type of response to amine [GO:0014075] Sources: GOC:mah Definition: Any process that results in a change in state or activity of a cell or an organism (in terms of movement, secretion, enzyme production, gene expression, etc.) as a result of a methylamine stimulus. Subtypes: GO:0036256